{
  "gene_symbol": "DEPDC4",
  "term_label": "Unknown molecular function",
  "gene_name": "DEP domain-containing protein 4",
  "gene": "UniProtKB:Q8N2C3",
  "term_id": "UNKNOWN:0001"
}